{
  "gene": "UniProtKB:P82663",
  "gene_symbol": "MRPS25",
  "term_id": "GO:0003735",
  "term_label": "structural constituent of ribosome",
  "gene_name": "Small ribosomal subunit protein mS25"
}